regulation of muscle tissue development [GO:1901861] (biological process) Definition: Any process that modulates the frequency, rate or extent of muscle tissue development. Relationships: is a type of regulation of developmental process [GO:0050793]; regulates muscle tissue development [GO:0060537] Subtypes: GO:0016202, negative regulation of muscle tissue development [GO:1901862], positive regulation of muscle tissue development [GO:1901863], regulation of smooth muscle tissue development [GO:1905899] References: PMID:23150719 Sources: GOC:TermGenie, GOC:yaf